{
  "gene_symbol": "EIF4EBP2",
  "term_label": "Unknown cellular component",
  "term_id": "UNKNOWN:0003",
  "gene": "UniProtKB:Q13542",
  "gene_name": "Eukaryotic translation initiation factor 4E-binding protein 2"
}